{
  "gene_name": "Aurora kinase B",
  "term_id": "GO:0032133",
  "term_label": "chromosome passenger complex",
  "gene": "UniProtKB:Q96GD4",
  "gene_symbol": "AURKB"
}